{
  "gene_name": "B-cell CLL_lymphoma 9-like protein",
  "term_id": "GO:0008013",
  "term_label": "beta-catenin binding",
  "gene": "UniProtKB:Q86UU0",
  "gene_symbol": "BCL9L"
}